{
  "term_label": "cell differentiation",
  "term_id": "GO:0030154",
  "gene_name": "Tomoregulin-2",
  "gene": "UniProtKB:Q9UIK5",
  "gene_symbol": "TMEFF2"
}